{
  "term_id": "GO:0015271",
  "term_label": "outward rectifier potassium channel activity",
  "gene": "UniProtKB:Q96T55",
  "gene_name": "Potassium channel subfamily K member 16",
  "gene_symbol": "KCNK16"
}